{
  "gene": "UniProtKB:Q9NR55",
  "gene_name": "Basic leucine zipper transcriptional factor ATF-like 3",
  "term_id": "GO:0000978",
  "gene_symbol": "BATF3",
  "term_label": "RNA polymerase II cis-regulatory region sequence-specific DNA binding"
}